{
  "term_id": "UNKNOWN:0003",
  "gene": "UniProtKB:Q8TCT1",
  "gene_name": "Phosphoethanolamine_phosphocholine phosphatase",
  "gene_symbol": "PHOSPHO1",
  "term_label": "Unknown cellular component"
}